dAMP metabolic process [GO:0046053] (biological process) Relationships: is a type of GO:0009151; is a type of purine deoxyribonucleoside monophosphate metabolic process [GO:0009170] Sources: GOC:go_curators Subtypes: dAMP biosynthetic process [GO:0006170], dAMP catabolic process [GO:0046059] Definition: The chemical reactions and pathways involving dAMP, deoxyadenosine monophosphate (2'-deoxyadenosine 5'-phosphate). Also known as: dAMP metabolism